negative regulation of meiosis I [GO:0110029] (biological process) Sources: GOC:vw Relationships: is a type of negative regulation of meiotic nuclear division [GO:0045835]; is a type of regulation of meiosis I [GO:0060631]; negatively regulates meiosis I [GO:0007127] Subtypes: GO:1905318 Definition: Any process that stops, prevents, or reduces the frequency, rate or extent of meiosis I, a cell cycle process comprising the steps by which a cell progresses through the first phase of meiosis, in which cells divide and homologous chromosomes are paired and segregated from each other, producing two daughter cells.